{
  "term_label": "DNA-binding transcription activator activity, RNA polymerase II-specific",
  "gene_name": "Transcription factor SOX-3",
  "term_id": "GO:0001228",
  "gene_symbol": "SOX3",
  "gene": "UniProtKB:P41225"
}